{
  "gene_name": "Rho GTPase-activating protein 36",
  "gene": "UniProtKB:Q6ZRI8",
  "term_label": "actin cytoskeleton",
  "gene_symbol": "ARHGAP36",
  "term_id": "GO:0015629"
}